{
  "gene": "UniProtKB:Q15084",
  "gene_symbol": "PDIA6",
  "term_label": "protein-disulfide reductase activity",
  "gene_name": "Protein disulfide-isomerase A6",
  "term_id": "GO:0015035"
}